sepal giant cell development [GO:0090393] (biological process) Relationships: is a type of cell development [GO:0048468]; is part of sepal giant cell differentiation [GO:0090392] Sources: GOC:tb Also known as: sepal giant cell formation Definition: The process aimed at the progression of a sepal giant cell over time, from initial commitment of the cell to a specific fate, to the fully functional differentiated cell.